positive regulation of transcription elongation by RNA polymerase II [GO:0032968] (biological process) Also known as: positive regulation of RNA elongation from RNA polymerase II promoter, positive regulation of transcription elongation from RNA polymerase II promoter, positive regulation of gene-specific transcription elongation from RNA polymerase II promoter Sources: GOC:mah, GOC:txnOH Relationships: is a type of positive regulation of DNA-templated transcription, elongation [GO:0032786]; is a type of GO:0034243; is a type of positive regulation of transcription by RNA polymerase II [GO:0045944]; positively regulates transcription elongation by RNA polymerase II [GO:0006368] Definition: Any process that activates or increases the frequency, rate or extent of transcription elongation, the extension of an RNA molecule after transcription initiation and promoter clearance by the addition of ribonucleotides, catalyzed by RNA polymerase II.